calcitonin catabolic process [GO:0010816] (BP) Relationships: is a type of GO:0042447; is a type of amide metabolic process [GO:0043603] Sources: GOC:BHF, GOC:rl Definition: The chemical reactions and pathways resulting in the breakdown of the peptide calcitonin.